{
  "term_label": "lymphocyte chemotaxis",
  "gene_symbol": "GPR15L",
  "gene_name": "Protein GPR15LG",
  "gene": "UniProtKB:Q6UWK7",
  "term_id": "GO:0048247"
}